{
  "term_id": "GO:0072518",
  "term_label": "Rho-dependent protein serine/threonine kinase activity",
  "gene_name": "Rho-associated protein kinase 1",
  "gene_symbol": "ROCK1",
  "gene": "UniProtKB:Q13464"
}